L-tyrosine biosynthetic process from chorismate via L-arogenate [GO:0033584] (biological process) Sources: GOC:mah Relationships: is a type of GO:0006571; is a type of chorismate metabolic process [GO:0046417] Definition: The chemical reactions and pathways resulting in the formation of L-tyrosine from other compounds, including chorismate, via the intermediate L-arogenate. Also known as: tyrosine biosynthetic process from chorismate via L-arogenate, L-tyrosine anabolism from chorismate via L-arogenate, L-tyrosine formation from chorismate via L-arogenate, L-tyrosine synthesis from chorismate via L-arogenate